{
  "gene": "UniProtKB:P37059",
  "term_label": "steroid metabolic process",
  "gene_symbol": "HSD17B2",
  "term_id": "GO:0008202",
  "gene_name": "17-beta-hydroxysteroid dehydrogenase type 2"
}